clathrin-sculpted glutamate transport vesicle membrane [GO:0060203] (cellular component) Relationships: is a type of transport vesicle membrane [GO:0030658]; is a type of clathrin-coated vesicle membrane [GO:0030665]; is part of clathrin-sculpted glutamate transport vesicle [GO:0060199] Sources: GOC:dph Also known as: clathrin sculpted glutamate constitutive secretory pathway transport vesicle membrane, clathrin sculpted glutamate transport vesicle membrane Definition: The lipid bilayer surrounding a clathrin-sculpted glutamate transport vesicle.